{
  "gene_name": "Synaptotagmin-9",
  "term_label": "plasma membrane",
  "gene_symbol": "SYT9",
  "term_id": "GO:0005886",
  "gene": "UniProtKB:Q86SS6"
}